{
  "gene_name": "DNA-directed RNA polymerases I and III subunit RPAC2",
  "term_id": "GO:0003899",
  "gene": "UniProtKB:P0DPB6",
  "term_label": "DNA-directed RNA polymerase activity",
  "gene_symbol": "POLR1D"
}